{
  "gene_name": "Multidrug and toxin extrusion protein 1",
  "gene_symbol": "SLC47A1",
  "term_label": "membrane",
  "term_id": "GO:0016020",
  "gene": "UniProtKB:Q96FL8"
}